subthalamic nucleus development [GO:0021763] (biological process) Also known as: corpus luysi development Sources: GOC:cls, GOC:dgh, GOC:dph, GOC:jid, GO_REF:0000021 Relationships: is a type of neural nucleus development [GO:0048857]; is part of subthalamus development [GO:0021539] Definition: The progression of the subthalamic nucleus over time from its initial formation until its mature state. The subthalamic nucleus is the lens-shaped nucleus located in the ventral part of the subthalamus on the inner aspect of the internal capsule that is concerned with the integration of somatic motor function.